{
  "gene": "UniProtKB:A0A1W2PRV1",
  "gene_name": "TATA-box-binding protein-associated factor 11-like protein 3",
  "term_id": "GO:0005669",
  "term_label": "transcription factor TFIID complex",
  "gene_symbol": "TAF11L3"
}